lipid droplet [GO:0005811] (cellular component) Note: Note that this term does not refer to vesicles, but instead to structures in which lipids do not necessarily form bilayers. Subtypes: ascus lipid droplet [GO:0005633], monolayer-surrounded lipid storage body [GO:0012511] Sources: GOC:mah, GOC:tb Definition: An intracellular non-membrane-bounded organelle comprising a matrix of coalesced lipids surrounded by a phospholipid monolayer. May include associated proteins. Also known as: adiposome, lipid body, lipid particle Relationships: is_a intracellular membraneless organelle [GO:0043232]